{
  "gene_symbol": "ITGB5",
  "gene_name": "Integrin beta-5",
  "term_id": "GO:0008305",
  "term_label": "integrin complex",
  "gene": "UniProtKB:P18084"
}